{
  "gene_name": "Beta-chimaerin",
  "term_label": "acrosome assembly",
  "term_id": "GO:0001675",
  "gene": "UniProtKB:P52757",
  "gene_symbol": "CHN2"
}